chorion micropyle formation [GO:0046844] (biological process) Sources: ISBN:0879694238 Relationships: is a type of developmental process involved in reproduction [GO:0003006]; is a type of anatomical structure formation involved in morphogenesis [GO:0048646]; is part of egg chorion assembly [GO:0007306] Definition: Establishment of the micropyle, a single cone-shaped specialization of the chorion that allows sperm entry into the egg prior to fertilization.